negative regulation of hepatocyte apoptotic process [GO:1903944] (biological process) Also known as: down regulation of hepatocyte apoptotic process, down-regulation of hepatocyte apoptotic process, downregulation of hepatocyte apoptotic process, down regulation of hepatocyte apoptosis, down-regulation of hepatocyte apoptosis, downregulation of hepatocyte apoptosis, inhibition of hepatocyte apoptosis, inhibition of hepatocyte apoptotic process, negative regulation of hepatocyte apoptosis Definition: Any process that stops, prevents or reduces the frequency, rate or extent of hepatocyte apoptotic process. References: PMID:8649852 Sources: GOC:TermGenie, GO_REF:0000058 Relationships: is a type of regulation of hepatocyte apoptotic process [GO:1903943]; is a type of GO:1904036; negatively regulates hepatocyte apoptotic process [GO:0097284]